{
  "gene_symbol": "TSPY1",
  "term_id": "GO:0042393",
  "gene_name": "Testis-specific Y-encoded protein 1",
  "term_label": "histone binding",
  "gene": "UniProtKB:Q01534"
}